positive regulation of autophagosome maturation [GO:1901098] (biological process) Also known as: activation of autophagosome maturation, positive regulation of autophagic vacuole fusion, positive regulation of autophagosome fusion, up regulation of autophagic vacuole fusion, up regulation of autophagic vacuole maturation, up regulation of autophagosome maturation, up-regulation of autophagic vacuole fusion, up-regulation of autophagic vacuole maturation, up-regulation of autophagosome maturation, upregulation of autophagic vacuole fusion, upregulation of autophagic vacuole maturation, upregulation of autophagosome maturation, activation of amphisome-lysosome fusion, activation of autolysosome formation, activation of autophagic vacuole fusion, activation of autophagic vacuole maturation, activation of fusion of autophagosome with lysosome, positive regulation of amphisome-lysosome fusion, positive regulation of autolysosome formation, positive regulation of fusion of autophagosome with lysosome, up regulation of amphisome-lysosome fusion, up regulation of autolysosome formation, up regulation of fusion of autophagosome with lysosome, up-regulation of amphisome-lysosome fusion, up-regulation of autolysosome formation, up-regulation of fusion of autophagosome with lysosome, upregulation of amphisome-lysosome fusion, upregulation of autolysosome formation, upregulation of fusion of autophagosome with lysosome Relationships: is a type of GO:0010638; is a type of positive regulation of macroautophagy [GO:0016239]; is a type of positive regulation of protein-containing complex disassembly [GO:0043243]; is_a regulation of autophagosome maturation [GO:1901096]; positively regulates autophagosome maturation [GO:0097352] Definition: Any process that activates or increases the frequency, rate or extent of autophagosome maturation. References: PMID:10436019, PMID:21383079 Sources: GOC:TermGenie, GOC:autophagy